{
  "gene_name": "Mitochondrial fission factor",
  "term_id": "GO:0005777",
  "term_label": "peroxisome",
  "gene": "UniProtKB:Q9GZY8",
  "gene_symbol": "MFF"
}